{
  "gene_symbol": "GRIN3B",
  "gene_name": "Glutamate receptor ionotropic, NMDA 3B",
  "gene": "UniProtKB:O60391",
  "term_id": "GO:0035235",
  "term_label": "ionotropic glutamate receptor signaling pathway"
}